{
  "gene_symbol": "FANCM",
  "term_label": "3'-5' DNA helicase activity",
  "term_id": "GO:0043138",
  "gene": "UniProtKB:Q8IYD8",
  "gene_name": "Fanconi anemia group M protein"
}